{
  "gene_symbol": "CCDC24",
  "term_id": "UNKNOWN:0001",
  "gene_name": "Coiled-coil domain-containing protein 24",
  "term_label": "Unknown molecular function",
  "gene": "UniProtKB:Q8N4L8"
}